{
  "gene": "UniProtKB:Q92609",
  "term_label": "retromer complex",
  "gene_symbol": "TBC1D5",
  "gene_name": "TBC1 domain family member 5",
  "term_id": "GO:0030904"
}